{
  "gene_name": "Decorin",
  "term_id": "UNKNOWN:0002",
  "term_label": "Unknown biological process",
  "gene": "UniProtKB:P07585",
  "gene_symbol": "DCN"
}